baruol synthase activity [GO:0080011] (molecular function) Definition: Catalysis of the reaction: (S)-2,3-epoxysqualene = baruol. Baruol is also known as D:B-Friedo-Baccharan-5,21-dien-3-ol. References: PMID:17705488 Sources: RHEA:31987 Relationships: is_a GO:0031559